{
  "gene": "UniProtKB:Q9HC35",
  "term_id": "UNKNOWN:0003",
  "gene_name": "Echinoderm microtubule-associated protein-like 4",
  "term_label": "Unknown cellular component",
  "gene_symbol": "EML4"
}